{
  "gene_name": "Protein ENTREP3",
  "gene_symbol": "ENTREP3",
  "term_label": "Unknown molecular function",
  "term_id": "UNKNOWN:0001",
  "gene": "UniProtKB:P81408"
}